{
  "gene_symbol": "KCNJ15",
  "term_label": "potassium ion import across plasma membrane",
  "gene": "UniProtKB:Q99712",
  "gene_name": "ATP-sensitive inward rectifier potassium channel 15",
  "term_id": "GO:1990573"
}